{
  "gene_name": "Run domain Beclin-1-interacting and cysteine-rich domain-containing protein",
  "gene": "UniProtKB:Q92622",
  "gene_symbol": "RUBCN",
  "term_id": "GO:1901097",
  "term_label": "negative regulation of autophagosome maturation"
}